RNA polymerase activity [GO:0097747] (molecular function) Regulation: negatively regulated by RNA polymerase inhibitor activity [GO:0140870]; negatively regulated by GO:0140871 Sources: GOC:pf Definition: Catalysis of the reaction: nucleoside triphosphate + RNA(n) = diphosphate + RNA(n+1); the synthesis of RNA from ribonucleotide triphosphates in the presence of a nucleic acid template. Subtypes: 5'-3' RNA polymerase activity [GO:0034062], 3'-5' RNA polymerase activity [GO:0097748] Relationships: is a type of nucleotidyltransferase activity [GO:0016779]; is a type of GO:0140098